{
  "gene": "UniProtKB:Q3C1V1",
  "gene_symbol": "C11orf91",
  "term_id": "UNKNOWN:0003",
  "gene_name": "Uncharacterized protein C11orf91",
  "term_label": "Unknown cellular component"
}